{
  "term_label": "ubiquitin protein ligase activity",
  "gene_symbol": "HECW2",
  "gene": "UniProtKB:Q9P2P5",
  "term_id": "GO:0061630",
  "gene_name": "E3 ubiquitin-protein ligase HECW2"
}